{
  "gene_name": "Beta-galactosidase-1-like protein 3",
  "term_label": "galactose catabolic process",
  "gene_symbol": "GLB1L3",
  "term_id": "GO:0019388",
  "gene": "UniProtKB:Q8NCI6"
}